alkylthioltransferase activity [GO:0050497] (molecular function) Definition: Catalysis of the transfer of an alkylthio group from one compound (donor) to another (acceptor). Relationships: is a type of GO:0016782 Sources: EC:2.8.4.-, GOC:ai Subtypes: methylthiotransferase activity [GO:0035596], coenzyme-B sulfoethylthiotransferase activity [GO:0050524], mycothiol-arsenate ligase activity [GO:0102100] Also known as: transferase activity, transferring alkylthio groups